{
  "term_label": "histone binding",
  "gene": "UniProtKB:P0CW00",
  "gene_symbol": "TSPY8",
  "term_id": "GO:0042393",
  "gene_name": "Testis-specific Y-encoded protein 8"
}